{
  "gene": "UniProtKB:O15156",
  "term_id": "GO:0010628",
  "gene_name": "Zinc finger and BTB domain-containing protein 7B",
  "term_label": "positive regulation of gene expression",
  "gene_symbol": "ZBTB7B"
}